{
  "term_label": "negative regulation of single stranded viral RNA replication via double stranded DNA intermediate",
  "gene_name": "DNA dC-dU-editing enzyme APOBEC-3B",
  "gene_symbol": "APOBEC3B",
  "gene": "UniProtKB:Q9UH17",
  "term_id": "GO:0045869"
}